{
  "term_label": "Unknown cellular component",
  "gene_symbol": "CACUL1",
  "term_id": "UNKNOWN:0003",
  "gene_name": "CDK2-associated and cullin domain-containing protein 1",
  "gene": "UniProtKB:Q86Y37"
}